{
  "gene": "UniProtKB:Q9BSH5",
  "gene_name": "Haloacid dehalogenase-like hydrolase domain-containing protein 3",
  "gene_symbol": "HDHD3",
  "term_label": "nucleus",
  "term_id": "GO:0005634"
}